{
  "gene_name": "Transmembrane 6 superfamily member 1",
  "term_label": "Unknown biological process",
  "gene_symbol": "TM6SF1",
  "gene": "UniProtKB:Q9BZW5",
  "term_id": "UNKNOWN:0002"
}